{
  "term_label": "release of sequestered calcium ion into cytosol",
  "gene_name": "Transient receptor potential cation channel subfamily M member 2",
  "gene_symbol": "TRPM2",
  "gene": "UniProtKB:O94759",
  "term_id": "GO:0051209"
}